positive regulation of ornithine catabolic process [GO:1903268] (BP) Definition: Any process that activates or increases the frequency, rate or extent of ornithine catabolic process. Also known as: positive regulation of ornithine breakdown, positive regulation of ornithine catabolism, positive regulation of ornithine degradation, up regulation of ornithine breakdown, up regulation of ornithine catabolic process, up regulation of ornithine catabolism, up regulation of ornithine degradation, up-regulation of ornithine breakdown, up-regulation of ornithine catabolic process, up-regulation of ornithine catabolism, up-regulation of ornithine degradation, upregulation of ornithine breakdown, upregulation of ornithine catabolic process, upregulation of ornithine catabolism, upregulation of ornithine degradation, activation of ornithine breakdown, activation of ornithine catabolic process, activation of ornithine catabolism, activation of ornithine degradation References: PMID:12679340 Sources: GOC:TermGenie, GOC:bhm, GO_REF:0000058 Relationships: is a type of positive regulation of catabolic process [GO:0009896]; is_a positive regulation of amino acid metabolic process [GO:0045764]; is a type of positive regulation of small molecule metabolic process [GO:0062013]; is a type of regulation of ornithine catabolic process [GO:1903266]; positively regulates L-ornithine catabolic process [GO:0006593]